{
  "gene_symbol": "GRIK1",
  "gene": "UniProtKB:P39086",
  "gene_name": "Glutamate receptor ionotropic, kainate 1",
  "term_id": "GO:0035249",
  "term_label": "synaptic transmission, glutamatergic"
}